alanyl aminopeptidase activity [GO:0016285] (molecular function) Definition: Catalysis of the release of an N-terminal amino acid, preferentially alanine, from a wide range of peptides, amides and arylamides. Also known as: aminopolypeptidase activity, cytosol alanyl aminopeptidase activity, arylamidase activity, cytosol aminopeptidase III activity, human liver aminopeptidase, liver aminopeptidase activity, membrane alanine aminopeptidase, membrane alanyl aminopeptidase, puromycin-sensitive aminopeptidase activity, soluble alanyl aminopeptidase activity, thiol-activated aminopeptidase activity Sources: EC:3.4.11.14 Relationships: is a type of aminopeptidase activity [GO:0004177]